{
  "term_label": "cytosol",
  "term_id": "GO:0005829",
  "gene": "UniProtKB:Q3YEC7",
  "gene_symbol": "RABL6",
  "gene_name": "Rab-like protein 6"
}